{
  "gene_symbol": "MTRNR2L6",
  "term_id": "UNKNOWN:0003",
  "gene_name": "Humanin-like 6",
  "gene": "UniProtKB:P0CJ73",
  "term_label": "Unknown cellular component"
}